positive regulation of microtubule nucleation [GO:0090063] (biological process) Subtypes: activation of microtubule nucleation [GO:0090064] Relationships: is a type of GO:0010968; is a type of positive regulation of microtubule polymerization [GO:0031116]; positively regulates microtubule nucleation [GO:0007020] Definition: Any process that increases the rate, frequency or extent of microtubule nucleation. Microtubule nucleation is the 'de novo' formation of a microtubule, in which tubulin heterodimers form metastable oligomeric aggregates, some of which go on to support formation of a complete microtubule. Microtubule nucleation usually occurs from a specific site within a cell. Sources: GOC:dph, GOC:tb